trichome patterning [GO:0048629] (biological process) Regulation: regulated by regulation of trichome patterning [GO:1900032]; negatively regulated by negative regulation of trichome patterning [GO:1900033] Also known as: trichome distribution, trichome pattern biosynthesis, trichome pattern formation, trichome spacing, trichome pattern specification Definition: The regionalization process of establishing the non-random spatial arrangement of trichomes on the surface and margin of a leaf. Process involves signaling between adjacent epidermal cells that results in differentiation of some epidermal cells into trichomes. References: PMID:10368181 Sources: GOC:jid, GOC:mtg_sensu, GOC:sm, GOC:tb, ISBN:0865427429 Relationships: is_a regionalization [GO:0003002]; is a type of cell-cell signaling involved in cell fate commitment [GO:0045168]; is part of trichome differentiation [GO:0010026]